{
  "gene_symbol": "CTSZ",
  "term_label": "proteolysis involved in protein catabolic process",
  "term_id": "GO:0051603",
  "gene": "UniProtKB:Q9UBR2",
  "gene_name": "Cathepsin Z"
}